{
  "gene_name": "Mitochondrial import receptor subunit TOM22 homolog",
  "gene_symbol": "TOMM22",
  "term_label": "mitochondrial outer membrane translocase complex",
  "term_id": "GO:0005742",
  "gene": "UniProtKB:Q9NS69"
}